{
  "term_label": "NuA4 histone acetyltransferase complex",
  "gene": "UniProtKB:Q9UBU8",
  "gene_symbol": "MORF4L1",
  "gene_name": "Mortality factor 4-like protein 1",
  "term_id": "GO:0035267"
}